{
  "term_id": "GO:0061630",
  "gene_name": "E3 ubiquitin-protein ligase RNF26",
  "term_label": "ubiquitin protein ligase activity",
  "gene_symbol": "RNF26",
  "gene": "UniProtKB:Q9BY78"
}